{
  "gene": "UniProtKB:Q92889",
  "term_label": "damaged DNA binding",
  "term_id": "GO:0003684",
  "gene_name": "DNA repair endonuclease XPF",
  "gene_symbol": "ERCC4"
}